PKM2 protein kinase complex [GO:1990360] (cellular component) Definition: A protein complex capable of phosphorylating a large number of protein targets. Contributes to cell proliferation under glycose starvation conditions. In human, the complex is present as a dimer. Relationships: is_a protein kinase complex [GO:1902911] Also known as: PKM2-SAICAR complex, PKM2-SAICAR protein kinase complex References: PMID:24606918 Sources: GOC:bhm